{
  "gene_name": "Golgin subfamily A member 2",
  "gene": "UniProtKB:Q08379",
  "term_label": "Golgi cisterna membrane",
  "gene_symbol": "GOLGA2",
  "term_id": "GO:0032580"
}